{
  "gene": "UniProtKB:P27986",
  "term_id": "GO:0046935",
  "gene_name": "Phosphatidylinositol 3-kinase regulatory subunit alpha",
  "term_label": "1-phosphatidylinositol-3-kinase regulator activity",
  "gene_symbol": "PIK3R1"
}